{
  "term_label": "RNA polymerase II cis-regulatory region sequence-specific DNA binding",
  "term_id": "GO:0000978",
  "gene_name": "Homeobox protein DLX-2",
  "gene_symbol": "DLX2",
  "gene": "UniProtKB:Q07687"
}